{
  "term_label": "Unknown molecular function",
  "gene": "UniProtKB:Q9BYQ8",
  "gene_name": "Keratin-associated protein 4-9",
  "term_id": "UNKNOWN:0001",
  "gene_symbol": "KRTAP4-9"
}